{
  "term_id": "GO:0007165",
  "gene_name": "Triggering receptor expressed on myeloid cells 2",
  "gene": "UniProtKB:Q9NZC2",
  "term_label": "signal transduction",
  "gene_symbol": "TREM2"
}